{
  "term_id": "UNKNOWN:0002",
  "term_label": "Unknown biological process",
  "gene": "UniProtKB:Q5THK1",
  "gene_name": "Protein PRR14L",
  "gene_symbol": "PRR14L"
}